{
  "gene": "UniProtKB:O43556",
  "term_label": "Unknown biological process",
  "gene_symbol": "SGCE",
  "gene_name": "Epsilon-sarcoglycan",
  "term_id": "UNKNOWN:0002"
}